formation by host of specialized structure for nutrient acquisition from symbiont [GO:0052098] (biological process) Definition: The assembly by an organism of a cellular component or anatomical structure for the purpose of obtaining nutrients from a symbiont organism. The symbiont is defined as the smaller of the organisms involved in a symbiotic interaction. Sources: GOC:mtg_pamgo_17jul06 Relationships: is a type of biological process involved in interaction with symbiont [GO:0051702]; is part of acquisition of nutrients from symbiont [GO:0051850]